{
  "term_id": "GO:0000122",
  "gene": "UniProtKB:P56693",
  "gene_symbol": "SOX10",
  "gene_name": "Transcription factor SOX-10",
  "term_label": "negative regulation of transcription by RNA polymerase II"
}